{
  "term_id": "GO:0045892",
  "term_label": "negative regulation of DNA-templated transcription",
  "gene_symbol": "KDM8",
  "gene_name": "Bifunctional peptidase and arginyl-hydroxylase JMJD5",
  "gene": "UniProtKB:Q8N371"
}